regulation of hemostasis [GO:1900046] (BP) Relationships: is a type of regulation of biological process [GO:0050789]; is a type of regulation of body fluid levels [GO:0050878]; RO_0002211 hemostasis [GO:0007599] Subtypes: regulation of blood coagulation [GO:0030193], negative regulation of hemostasis [GO:1900047], positive regulation of hemostasis [GO:1900048] Definition: Any process that modulates the frequency, rate or extent of hemostasis. Sources: GOC:TermGenie